{
  "gene_symbol": "SPATA16",
  "term_label": "Unknown molecular function",
  "term_id": "UNKNOWN:0001",
  "gene_name": "Spermatogenesis-associated protein 16",
  "gene": "UniProtKB:Q9BXB7"
}